ARC complex [GO:0033167] (cellular component) Definition: A ribonucleoprotein complex that contains members of the Argonaute family of proteins, additional protein subunits, and duplex siRNA; required for heterochromatin assembly and siRNA generation. Possibly involved in the conversion of ds siRNA to ss siRNA. Relationships: is a type of RNAi effector complex [GO:0031332]; is a type of GO:0140513 References: PMID:17310250 Sources: GOC:vw Also known as: argonaute siRNA chaperone complex